{
  "gene": "UniProtKB:P50213",
  "gene_symbol": "IDH3A",
  "term_label": "tricarboxylic acid cycle",
  "term_id": "GO:0006099",
  "gene_name": "Isocitrate dehydrogenase [NAD] subunit alpha, mitochondrial"
}